{
  "term_id": "UNKNOWN:0001",
  "gene": "UniProtKB:Q9P0S3",
  "gene_symbol": "ORMDL1",
  "term_label": "Unknown molecular function",
  "gene_name": "ORM1-like protein 1"
}